lobar bronchus mesenchyme development [GO:0060483] (biological process) Relationships: is_a GO:0060484; is part of lobar bronchus development [GO:0060482] Definition: The biological process whose specific outcome is the progression of a lobar bronchus mesenchyme from an initial condition to its mature state. This process begins with the formation of the lobar bronchus mesenchyme and ends with the mature structure. The lobar bronchus mesenchyme is the mass of tissue composed of mesenchymal cells in the lobar bronchus. Sources: GOC:dph, GOC:mtg_lung